{
  "gene": "UniProtKB:P63261",
  "gene_symbol": "ACTG1",
  "gene_name": "Actin, cytoplasmic 2",
  "term_label": "NuA4 histone acetyltransferase complex",
  "term_id": "GO:0035267"
}